{
  "term_id": "GO:0005829",
  "term_label": "cytosol",
  "gene": "UniProtKB:P11086",
  "gene_name": "Phenylethanolamine N-methyltransferase",
  "gene_symbol": "PNMT"
}